{
  "term_label": "pericentriolar material",
  "term_id": "GO:0000242",
  "gene": "UniProtKB:Q8N4C6",
  "gene_name": "Ninein",
  "gene_symbol": "NIN"
}